{
  "gene": "UniProtKB:Q03167",
  "gene_symbol": "TGFBR3",
  "term_id": "GO:0050431",
  "term_label": "transforming growth factor beta binding",
  "gene_name": "Transforming growth factor beta receptor type 3"
}